{
  "gene": "UniProtKB:Q8NGK4",
  "term_label": "plasma membrane",
  "term_id": "GO:0005886",
  "gene_name": "Olfactory receptor 52K1",
  "gene_symbol": "OR52K1"
}